telomere cap complex [GO:0000782] (cellular component) Sources: GOC:elh Subtypes: nuclear telomere cap complex [GO:0000783], Tpg-containing telomere binding complex [GO:0043769] Note: Note that this term can be used in place of the obsolete cellular component term 'telomere ; GO:0005696'. Use with caution because this term refers to a specific protein complex and not a region of the chromosome. Relationships: is a type of protein-DNA complex [GO:0032993]; is part of chromosome, telomeric repeat region [GO:0140445] Definition: A complex of DNA and protein located at the end of a linear chromosome that protects and stabilizes a linear chromosome.